voltage-gated monoatomic ion channel activity [GO:0005244] (molecular function) Also known as: voltage-gated ion channel activity, voltage gated ion channel activity, voltage-dependent ion channel activity Relationships: is_a monoatomic ion channel activity [GO:0005216]; is a type of voltage-gated channel activity [GO:0022832] Definition: Enables the transmembrane transfer of an ion by a voltage-gated channel. An ion is an atom or group of atoms carrying an electric charge by virtue of having gained or lost one or more electrons. A voltage-gated channel is a channel whose open state is dependent on the voltage across the membrane in which it is embedded. Subtypes: GO:0004972, voltage-gated monoatomic anion channel activity [GO:0008308], voltage-gated monoatomic cation channel activity [GO:0022843], voltage-gated monoatomic ion channel activity involved in regulation of presynaptic membrane potential [GO:0099508], voltage-gated monoatomic ion channel activity involved in regulation of postsynaptic membrane potential [GO:1905030] Sources: GOC:mtg_transport, ISBN:0198506732, ISBN:0815340729